{
  "gene": "UniProtKB:O15231",
  "gene_symbol": "ZNF185",
  "term_label": "Unknown biological process",
  "gene_name": "Zinc finger protein 185",
  "term_id": "UNKNOWN:0002"
}